{
  "term_label": "peripheral nervous system myelin formation",
  "term_id": "GO:0032290",
  "gene_name": "Noncompact myelin-associated protein",
  "gene_symbol": "NCMAP",
  "gene": "UniProtKB:Q5T1S8"
}